{
  "term_id": "UNKNOWN:0001",
  "gene_symbol": "C2CD4B",
  "gene_name": "C2 calcium-dependent domain-containing protein 4B",
  "term_label": "Unknown molecular function",
  "gene": "UniProtKB:A6NLJ0"
}